{
  "gene_name": "Cytoplasmic protein NCK1",
  "term_label": "cell migration",
  "term_id": "GO:0016477",
  "gene": "UniProtKB:P16333",
  "gene_symbol": "NCK1"
}